{
  "gene_name": "Bis(5'-adenosyl)-triphosphatase ENPP4",
  "gene_symbol": "ENPP4",
  "term_id": "GO:0047710",
  "term_label": "bis(5'-adenosyl)-triphosphatase activity",
  "gene": "UniProtKB:Q9Y6X5"
}